{
  "term_id": "GO:0005634",
  "term_label": "nucleus",
  "gene_name": "Forkhead box protein P1",
  "gene_symbol": "FOXP1",
  "gene": "UniProtKB:Q9H334"
}